{
  "term_id": "UNKNOWN:0002",
  "gene": "UniProtKB:O75072",
  "gene_name": "Ribitol-5-phosphate transferase FKTN",
  "gene_symbol": "FKTN",
  "term_label": "Unknown biological process"
}